positive regulation of spindle attachment to meiosis I kinetochore [GO:1904968] (biological process) Relationships: is a type of positive regulation of attachment of spindle microtubules to kinetochore [GO:0051987]; is_a regulation of spindle attachment to meiosis I kinetochore [GO:1904967]; is a type of GO:2000243; RO_0002213 spindle attachment to meiosis I kinetochore [GO:0051455] Also known as: positive regulation of attachment of spindle microtubules to kinetochore involved in homologous chromosome segregation, positive regulation of attachment of spindle microtubules to kinetochore involved in meiosis I, positive regulation of monopolar attachment, positive regulation of sister kinetochore mono-orientation, up regulation of attachment of spindle microtubules to kinetochore involved in homologous chromosome segregation, up regulation of attachment of spindle microtubules to kinetochore involved in meiosis I, up regulation of monopolar attachment, up regulation of sister kinetochore mono-orientation, up-regulation of attachment of spindle microtubules to kinetochore involved in homologous chromosome segregation, up-regulation of attachment of spindle microtubules to kinetochore involved in meiosis I, up-regulation of monopolar attachment, up-regulation of sister kinetochore mono-orientation, upregulation of attachment of spindle microtubules to kinetochore involved in homologous chromosome segregation, upregulation of attachment of spindle microtubules to kinetochore involved in meiosis I, upregulation of monopolar attachment, upregulation of sister kinetochore mono-orientation, activation of attachment of spindle microtubules to kinetochore involved in homologous chromosome segregation, activation of attachment of spindle microtubules to kinetochore involved in meiosis I, activation of monopolar attachment, activation of sister kinetochore mono-orientation, activation of attachment of spindle microtubules to kinetochore during meiosis I, positive regulation of attachment of spindle microtubules to kinetochore during meiosis I, up regulation of attachment of spindle microtubules to kinetochore during meiosis I, up-regulation of attachment of spindle microtubules to kinetochore during meiosis I, upregulation of attachment of spindle microtubules to kinetochore during meiosis I Definition: Any process that activates or increases the frequency, rate or extent of attachment of spindle microtubules to kinetochore involved in homologous chromosome segregation. References: PMID:23770679 Sources: GOC:TermGenie, GO_REF:0000058